{
  "gene": "UniProtKB:Q96B70",
  "gene_name": "Leukocyte receptor cluster member 9",
  "gene_symbol": "LENG9",
  "term_label": "Unknown molecular function",
  "term_id": "UNKNOWN:0001"
}